positive regulation of organelle assembly [GO:1902117] (biological process) Sources: GOC:TermGenie, GOC:pr Subtypes: positive regulation of cytoplasmic mRNA processing body assembly [GO:0010606], positive regulation of cilium assembly [GO:0045724], positive regulation of centriole replication [GO:0046601], positive regulation of stress granule assembly [GO:0062029], positive regulation of pseudohyphal septin ring assembly [GO:0062165], GO:0071803, positive regulation of postsynaptic density assembly [GO:0160036], positive regulation of cellulosome assembly [GO:1900505], positive regulation of bacterial-type flagellum assembly [GO:1902210], GO:1903553, GO:1904757, positive regulation of cardiac myofibril assembly [GO:1905306], positive regulation of kinetochore assembly [GO:1905561], positive regulation of spindle assembly [GO:1905832], positive regulation of autophagosome assembly [GO:2000786] Relationships: is a type of positive regulation of organelle organization [GO:0010638]; is a type of positive regulation of cellular component biogenesis [GO:0044089]; is a type of GO:1902115; positively regulates organelle assembly [GO:0070925] Also known as: up regulation of organelle assembly, up-regulation of organelle assembly, upregulation of organelle assembly, activation of organelle assembly Definition: Any process that activates or increases the frequency, rate or extent of organelle assembly.